{
  "term_id": "UNKNOWN:0002",
  "gene_name": "UPF0450 protein C17orf58",
  "gene": "UniProtKB:Q2M2W7",
  "gene_symbol": "C17orf58",
  "term_label": "Unknown biological process"
}